{
  "gene": "UniProtKB:Q9BV19",
  "term_id": "UNKNOWN:0003",
  "term_label": "Unknown cellular component",
  "gene_name": "Uncharacterized protein C1orf50",
  "gene_symbol": "C1orf50"
}